{
  "gene_name": "Suppressor of cytokine signaling 1",
  "gene_symbol": "SOCS1",
  "term_label": "cytokine receptor binding",
  "term_id": "GO:0005126",
  "gene": "UniProtKB:O15524"
}